{
  "gene": "UniProtKB:O15034",
  "term_label": "neuromuscular synaptic transmission",
  "term_id": "GO:0007274",
  "gene_symbol": "RIMBP2",
  "gene_name": "RIMS-binding protein 2"
}